alpha-beta T cell receptor complex [GO:0042105] (cellular component) Definition: A T cell receptor complex in which the TCR heterodimer comprises alpha and beta chains, associated with the CD3 complex; recognizes a complex consisting of an antigen-derived peptide bound to a class I or class II MHC protein. Also known as: alpha-beta T lymphocyte receptor complex, alpha-beta T-cell receptor complex, alpha-beta T-lymphocyte receptor complex, alpha-beta TCR complex Sources: GOC:mah, ISBN:0781735149 Relationships: is a type of T cell receptor complex [GO:0042101]